{
  "gene_name": "Nck-associated protein 5-like",
  "term_label": "microtubule bundle formation",
  "term_id": "GO:0001578",
  "gene": "UniProtKB:Q9HCH0",
  "gene_symbol": "NCKAP5L"
}